{
  "term_label": "cellular response to glucose stimulus",
  "gene_name": "Phosphoenolpyruvate carboxykinase, cytosolic [GTP]",
  "gene": "UniProtKB:P35558",
  "gene_symbol": "PCK1",
  "term_id": "GO:0071333"
}